{
  "gene": "UniProtKB:Q8N339",
  "term_id": "GO:0006882",
  "gene_name": "Metallothionein-1M",
  "gene_symbol": "MT1M",
  "term_label": "intracellular zinc ion homeostasis"
}